{
  "gene_symbol": "ROCK2",
  "term_label": "regulation of cell junction assembly",
  "gene_name": "Rho-associated protein kinase 2",
  "gene": "UniProtKB:O75116",
  "term_id": "GO:1901888"
}